{
  "gene": "UniProtKB:Q5JNZ5",
  "term_label": "Unknown biological process",
  "gene_name": "Putative ribosomal protein eS26-like",
  "term_id": "UNKNOWN:0002",
  "gene_symbol": "RPS26P11"
}